{
  "gene": "UniProtKB:P48634",
  "gene_symbol": "PRRC2A",
  "term_id": "UNKNOWN:0001",
  "term_label": "Unknown molecular function",
  "gene_name": "Protein PRRC2A"
}